{
  "gene_name": "RWD domain-containing protein 2B",
  "gene": "UniProtKB:P57060",
  "gene_symbol": "RWDD2B",
  "term_label": "Unknown cellular component",
  "term_id": "UNKNOWN:0003"
}